{
  "gene_symbol": "RNF185",
  "gene_name": "E3 ubiquitin-protein ligase RNF185",
  "gene": "UniProtKB:Q96GF1",
  "term_label": "ubiquitin-like protein conjugating enzyme binding",
  "term_id": "GO:0044390"
}